{
  "gene": "UniProtKB:Q16637",
  "gene_name": "Survival motor neuron protein",
  "term_id": "GO:0000387",
  "term_label": "spliceosomal snRNP assembly",
  "gene_symbol": "SMN2"
}